{
  "gene_symbol": "HRH3",
  "term_label": "G protein-coupled receptor signaling pathway, coupled to cyclic nucleotide second messenger",
  "gene": "UniProtKB:Q9Y5N1",
  "gene_name": "Histamine H3 receptor",
  "term_id": "GO:0007187"
}